{
  "gene_name": "LHFPL tetraspan subfamily member 5 protein",
  "gene_symbol": "LHFPL5",
  "gene": "UniProtKB:Q8TAF8",
  "term_id": "GO:0007605",
  "term_label": "sensory perception of sound"
}